{
  "term_id": "GO:0006357",
  "gene_symbol": "ZBTB7B",
  "gene_name": "Zinc finger and BTB domain-containing protein 7B",
  "gene": "UniProtKB:O15156",
  "term_label": "regulation of transcription by RNA polymerase II"
}